{
  "gene_name": "Homeobox protein Nkx-2.3",
  "gene": "UniProtKB:Q8TAU0",
  "gene_symbol": "NKX2-3",
  "term_label": "cell differentiation",
  "term_id": "GO:0030154"
}